{
  "gene_symbol": "TVP23B",
  "gene": "UniProtKB:Q9NYZ1",
  "term_label": "protein secretion",
  "gene_name": "Golgi apparatus membrane protein TVP23 homolog B",
  "term_id": "GO:0009306"
}